{
  "gene": "UniProtKB:Q86WA8",
  "gene_name": "Lon protease homolog 2, peroxisomal",
  "gene_symbol": "LONP2",
  "term_label": "Unknown molecular function",
  "term_id": "UNKNOWN:0001"
}